{
  "gene_symbol": "LMO1",
  "gene": "UniProtKB:P25800",
  "gene_name": "Rhombotin-1",
  "term_label": "transcription coactivator activity",
  "term_id": "GO:0003713"
}